ATPase-coupled phosphate ion transmembrane transporter activity [GO:0015415] (molecular function) Relationships: is a type of GO:0005315; is a type of ATPase-coupled transmembrane transporter activity [GO:0042626] Definition: Enables the transfer of a solute or solutes from one side of a membrane to the other according to the reaction: ATP + H2O + phosphate(out) = ADP + phosphate + phosphate(in). Sources: EC:7.3.2.1 Also known as: phosphate porter activity, phosphate transporting ATPase activity, ABC phosphate transporter activity, phosphate ABC transporter, ATP phosphohydrolase (phosphate-importing), phosphate ion transmembrane-transporting ATPase activity, phosphate-transporting ATPase activity